{
  "gene": "UniProtKB:O75509",
  "term_label": "neuron apoptotic process",
  "gene_name": "Tumor necrosis factor receptor superfamily member 21",
  "gene_symbol": "TNFRSF21",
  "term_id": "GO:0051402"
}